{
  "term_label": "proteasome core complex, beta-subunit complex",
  "term_id": "GO:0019774",
  "gene_symbol": "PSMB9",
  "gene_name": "Proteasome subunit beta type-9",
  "gene": "UniProtKB:P28065"
}